{
  "term_label": "Unknown molecular function",
  "gene": "UniProtKB:O15164",
  "term_id": "UNKNOWN:0001",
  "gene_symbol": "TRIM24",
  "gene_name": "Transcription intermediary factor 1-alpha"
}